{
  "gene_name": "Small ribosomal subunit protein uS11m",
  "gene_symbol": "MRPS11",
  "term_id": "GO:0006412",
  "term_label": "translation",
  "gene": "UniProtKB:P82912"
}